{
  "gene_name": "Putative uncharacterized protein encoded by LINC01556",
  "term_id": "UNKNOWN:0002",
  "term_label": "Unknown biological process",
  "gene_symbol": "LINC01556",
  "gene": "UniProtKB:Q5JQF7"
}